{
  "gene_name": "MAM and LDL-receptor class A domain-containing protein 1",
  "gene": "UniProtKB:Q5VYJ5",
  "term_id": "UNKNOWN:0002",
  "gene_symbol": "MALRD1",
  "term_label": "Unknown biological process"
}